{
  "gene_symbol": "FAM181A",
  "gene_name": "Protein FAM181A",
  "term_id": "UNKNOWN:0003",
  "gene": "UniProtKB:Q8N9Y4",
  "term_label": "Unknown cellular component"
}